{
  "gene_name": "Olfactory receptor 51B6",
  "gene": "UniProtKB:Q9H340",
  "gene_symbol": "OR51B6",
  "term_id": "GO:0004984",
  "term_label": "olfactory receptor activity"
}